cell wall modification involved in multidimensional cell growth [GO:0042547] (biological process) Sources: GOC:dph, GOC:jl, GOC:tb Subtypes: GO:0009831 Definition: The series of events resulting in chemical or structural changes to existing cell walls and contribute to multidimensional cell growth. Also known as: cell wall modification during cell expansion, cell wall modification during multidimensional cell growth Relationships: is a type of cell wall modification [GO:0042545]; is part of multidimensional cell growth [GO:0009825]